{
  "gene_symbol": "STAMBP",
  "term_label": "cleavage furrow",
  "term_id": "GO:0032154",
  "gene": "UniProtKB:O95630",
  "gene_name": "STAM-binding protein"
}